{
  "gene": "UniProtKB:Q96G74",
  "term_label": "positive regulation of TORC2 signaling",
  "gene_name": "OTU domain-containing protein 5",
  "term_id": "GO:1904515",
  "gene_symbol": "OTUD5"
}